plasma membrane light-harvesting complex [GO:0030077] (cellular component) Subtypes: GO:0030078, light-harvesting complex, peripheral complex [GO:0030079] Relationships: is a type of GO:0030076; is part of GO:0031410; is part of plasma membrane-derived chromatophore [GO:0042716] Sources: GOC:mah, GOC:mtg_sensu Definition: A plasma membrane protein-pigment complex that may be closely or peripherally associated to photosynthetic reaction centers that participate in harvesting and transferring radiant energy to the reaction center. Examples of this complex are found in bacterial species.